{
  "gene_name": "Collagen alpha-1(XXIV) chain",
  "term_id": "GO:0030020",
  "term_label": "extracellular matrix structural constituent conferring tensile strength",
  "gene_symbol": "COL24A1",
  "gene": "UniProtKB:Q17RW2"
}